symbiont-mediated activation of host NF-kappaB cascade [GO:0085033] (biological process) References: PMID:11907233, PMID:17490702, PMID:21098302, PMID:21199955, PMID:31311877, PMID:7845680 Also known as: activation by symbiont of host I-kappaB kinase/NF-kappaB cascade, induction by symbiont of host I-kappaB kinase/NF-kappaB cascade, induction of host I-kappaB kinase/NF-kappaB cascade, induction of host canonical NF-kappaB signal transduction, positive regulation by symbiont of host I-kappaB kinase/NF-kappaB cascade, positive regulation by symbiont of host NF-kappaB-mediated signal transduction pathway, stimulation by symbiont of host I-kappaB kinase/NF-kappaB cascade, symbiont-mediated activation of host NF-kappaB signal transduction, up regulation by symbiont of host I-kappaB kinase/NF-kappaB cascade, up-regulation by symbiont of host I-kappaB kinase/NF-kappaB cascade, upregulation by symbiont of host I-kappaB kinase/NF-kappaB cascade, symbiont-mediated activation of host canonical NF-kappaB signal transduction Definition: A process that initiates, promotes, or enhances a host NF-kappaB-mediated signaling cascade. The host is defined as the larger of the organisms involved in a symbiotic interaction. Relationships: is a type of symbiont-mediated activation of host signal transduction pathway [GO:0052028]; is a type of symbiont-mediated perturbation of host NF-kappaB cascade [GO:0085032]